negative regulation of heptasaccharide transport [GO:1900295] (biological process) Relationships: is a type of GO:0051051; is a type of regulation of heptasaccharide transport [GO:1900294]; RO_0002212 GO:2001104 Definition: Any process that stops, prevents or reduces the frequency, rate or extent of heptasaccharide transport. Subtypes: negative regulation of maltoheptaose transport [GO:1900307] Sources: GOC:TermGenie, GOC:mengo_curators Also known as: down regulation of heptasaccharide transport, down-regulation of heptasaccharide transport, downregulation of heptasaccharide transport, inhibition of heptasaccharide transport